cell adhesion molecule production [GO:0060352] (biological process) Relationships: is a type of GO:0009987 Regulation: regulated by regulation of cell adhesion molecule production [GO:0060353]; negatively regulated by GO:0060354; positively regulated by GO:0060355 Sources: GOC:BHF, GOC:rl Definition: The appearance of a cell adhesion molecule due to biosynthesis or secretion.